{
  "gene": "UniProtKB:Q8IWF2",
  "term_id": "GO:0005788",
  "term_label": "endoplasmic reticulum lumen",
  "gene_symbol": "FOXRED2",
  "gene_name": "FAD-dependent oxidoreductase domain-containing protein 2"
}